{
  "gene_name": "Regulator of G-protein signaling 11",
  "term_label": "cytoplasm",
  "gene": "UniProtKB:O94810",
  "term_id": "GO:0005737",
  "gene_symbol": "RGS11"
}